conditioned taste aversion [GO:0001661] (biological process) References: PMID:9920659 Sources: GOC:dph Relationships: is a type of GO:0007631; is a type of associative learning [GO:0008306] Definition: A conditioned aversion to a specific chemical compound as a result of that compound being coupled with a noxious stimulus.